negative regulation of macrophage inflammatory protein-1 gamma production [GO:0071647] (biological process) Also known as: negative regulation of CCL9 production, negative regulation of MIP-1g production, negative regulation of chemokine (C-C motif) ligand 9 production Definition: Any process that stops, prevents, or reduces the frequency, rate, or extent of production of macrophage inflammatory protein-1 gamma. Relationships: is a type of GO:0032682; is a type of regulation of macrophage inflammatory protein-1 gamma production [GO:0071646]; negatively regulates macrophage inflammatory protein-1 gamma production [GO:0071607] Sources: GOC:mah